interleukin-5 production [GO:0032634] (biological process) Sources: GOC:mah Definition: The appearance of interleukin-5 due to biosynthesis or secretion following a cellular stimulus, resulting in an increase in its intracellular or extracellular levels. Regulation: regulated by regulation of interleukin-5 production [GO:0032674]; negatively regulated by negative regulation of interleukin-5 production [GO:0032714]; positively regulated by positive regulation of interleukin-5 production [GO:0032754] Also known as: IL-5 production, interleukin-5 biosynthetic process, interleukin-5 secretion Relationships: is_a GO:0001816